{
  "term_id": "GO:0005829",
  "gene_name": "Ras GTPase-activating protein-binding protein 2",
  "gene_symbol": "G3BP2",
  "term_label": "cytosol",
  "gene": "UniProtKB:Q9UN86"
}